{
  "term_label": "delta(3,5)-delta(2,4)-dienoyl-CoA isomerase activity",
  "term_id": "GO:0051750",
  "gene_name": "Delta(3,5)-Delta(2,4)-dienoyl-CoA isomerase, mitochondrial",
  "gene_symbol": "ECH1",
  "gene": "UniProtKB:Q13011"
}